{
  "term_id": "UNKNOWN:0003",
  "gene": "UniProtKB:Q8TEY7",
  "gene_name": "Ubiquitin carboxyl-terminal hydrolase 33",
  "gene_symbol": "USP33",
  "term_label": "Unknown cellular component"
}